{
  "gene_name": "Pleckstrin homology domain-containing family H member 1",
  "term_id": "UNKNOWN:0003",
  "gene": "UniProtKB:Q9ULM0",
  "term_label": "Unknown cellular component",
  "gene_symbol": "PLEKHH1"
}